positive regulation of peripheral tolerance induction [GO:0002660] (biological process) Subtypes: positive regulation of tolerance induction to tumor cell [GO:0002845], positive regulation of peripheral T cell tolerance induction [GO:0002851], positive regulation of peripheral B cell deletion [GO:0002910], positive regulation of peripheral B cell anergy [GO:0002919] Definition: Any process that activates or increases the frequency, rate, or extent of peripheral tolerance induction. Relationships: is a type of GO:0002654; is a type of regulation of peripheral tolerance induction [GO:0002658]; positively regulates peripheral tolerance induction [GO:0002465] Sources: GOC:add Also known as: up regulation of peripheral tolerance induction, up-regulation of peripheral tolerance induction, upregulation of peripheral tolerance induction, activation of peripheral tolerance induction, stimulation of peripheral tolerance induction